{
  "gene_symbol": "SSBP4",
  "gene_name": "Single-stranded DNA-binding protein 4",
  "term_id": "GO:0005634",
  "term_label": "nucleus",
  "gene": "UniProtKB:Q9BWG4"
}